{
  "gene_symbol": "SLCO1C1",
  "term_label": "bile acid and bile salt transport",
  "gene": "UniProtKB:Q9NYB5",
  "gene_name": "Solute carrier organic anion transporter family member 1C1",
  "term_id": "GO:0015721"
}